mesenchymal cell apoptotic process involved in metanephric nephron morphogenesis [GO:1901147] (biological process) Relationships: is a type of mesenchymal cell apoptotic process involved in metanephros development [GO:1900200]; is a type of mesenchymal cell apoptotic process involved in nephron morphogenesis [GO:1901145]; is part of GO:0072273 Regulation: regulated by regulation of mesenchymal cell apoptotic process involved in metanephric nephron morphogenesis [GO:0072304]; negatively regulated by negative regulation of mesenchymal cell apoptotic process involved in metanephric nephron morphogenesis [GO:0072305]; positively regulated by positive regulation of mesenchymal cell apoptotic process involved in metanephric nephron morphogenesis [GO:0072306] Sources: GOC:TermGenie, GOC:mtg_apoptosis Definition: Any mesenchymal cell apoptotic process that is involved in metanephric nephron morphogenesis.